dihydroflavanol 4-reductase activity [GO:0045552] (molecular function) Sources: RHEA:54444 Relationships: is a type of oxidoreductase activity, acting on the CH-OH group of donors, NAD or NADP as acceptor [GO:0016616] Also known as: NADPH-dihydromyricetin reductase activity, cis-3,4-leucopelargonidin:NADP+ 4-oxidoreductase activity, dihydroflavonol 4-reductase activity, dihydrokaempferol 4-reductase activity, dihydromyricetin reductase activity, dihydroquercetin reductase activity Definition: Catalysis of the reaction: a (2R,3S,4S)-leucoanthocyanidin + NADP+ = a (2R,3R)-dihydroflavonol + NADPH + H+.